{
  "term_label": "structural constituent of ribosome",
  "gene_name": "Small ribosomal subunit protein uS7",
  "gene_symbol": "RPS5",
  "gene": "UniProtKB:P46782",
  "term_id": "GO:0003735"
}